{
  "gene_symbol": "HNRNPM",
  "gene_name": "Heterogeneous nuclear ribonucleoprotein M",
  "term_label": "Unknown biological process",
  "gene": "UniProtKB:P52272",
  "term_id": "UNKNOWN:0002"
}